protein serine/threonine kinase activity [GO:0004674] (molecular function) Subtypes: transmembrane receptor protein serine/threonine kinase activity [GO:0004675], 3-phosphoinositide-dependent protein kinase activity [GO:0004676], DNA-dependent protein kinase activity [GO:0004677], GO:0004679, GO:0004683, GO:0004687, GO:0004690, cyclin-dependent protein serine/threonine kinase activity [GO:0004693], eukaryotic translation initiation factor 2alpha kinase activity [GO:0004694], diacylglycerol-dependent serine/threonine kinase activity [GO:0004697], GO:0004703, MAP kinase activity [GO:0004707], MAP kinase kinase kinase activity [GO:0004709], ribosomal protein S6 kinase activity [GO:0004711], GO:0004740, GO:0008349, RNA polymerase II CTD heptapeptide repeat kinase activity [GO:0008353], IkappaB kinase activity [GO:0008384], calcium-dependent protein serine/threonine kinase activity [GO:0009931], GO:0033867, GTP-dependent protein kinase activity [GO:0034211], histone H3S10 kinase activity [GO:0035175], GO:0035402, histone H3T6 kinase activity [GO:0035403], histone H2AXS139 kinase activity [GO:0035979], histone H3S28 kinase activity [GO:0044022], histone H4S1 kinase activity [GO:0044023], histone H2AS1 kinase activity [GO:0044024], histone H2BS14 kinase activity [GO:0044025], [hydroxymethylglutaryl-CoA reductase (NADPH)] kinase activity [GO:0047322], [3-methyl-2-oxobutanoate dehydrogenase (acetyl-transferring)] kinase activity [GO:0047323], tau-protein kinase activity [GO:0050321], [tyrosine 3-monooxygenase] kinase activity [GO:0050369], histone H3T3 kinase activity [GO:0072354], Rho-dependent protein serine/threonine kinase activity [GO:0072518], histone H1-4S187 kinase activity [GO:0140191], histone H1-4S27 kinase activity [GO:0140197], histone H1-4S35 kinase activity [GO:0140198], histone H2BS36 kinase activity [GO:0140823], histone H3S57 kinase activity [GO:0140855], histone H3T45 kinase activity [GO:0140857], histone H2AT120 kinase activity [GO:1990244] Also known as: protein serine kinase activity, protein threonine kinase activity, protein-serine kinase activity, serine kinase activity, serine protein kinase activity, serine-specific protein kinase activity, threonine-specific protein kinase activity, protein serine-threonine kinase activity, serine(threonine) protein kinase activity, serine/threonine protein kinase activity Relationships: is a type of GO:0004672 References: PMID:2956925 Sources: EC:2.7.11.-, GOC:bf Regulation: negatively regulated by protein serine/threonine kinase inhibitor activity [GO:0030291]; positively regulated by protein serine/threonine kinase activator activity [GO:0043539]; RO_0002211 by GO:0071900; negatively regulated by GO:0071901; positively regulated by positive regulation of protein serine/threonine kinase activity [GO:0071902] Definition: Catalysis of the reactions: ATP + protein serine = ADP + protein serine phosphate, and ATP + protein threonine = ADP + protein threonine phosphate.